{
  "gene": "UniProtKB:O75425",
  "term_id": "UNKNOWN:0001",
  "gene_name": "Motile sperm domain-containing protein 3",
  "gene_symbol": "MOSPD3",
  "term_label": "Unknown molecular function"
}